{
  "gene_symbol": "FAU",
  "term_label": "nucleus",
  "gene_name": "Ubiquitin-like FUBI-ribosomal protein eS30 fusion protein",
  "term_id": "GO:0005634",
  "gene": "UniProtKB:P62861"
}